glutamate:gamma-aminobutyric acid antiporter activity [GO:0070909] (molecular function) Sources: GOC:dh Relationships: is a type of gamma-aminobutyric acid transmembrane transporter activity [GO:0015185]; is_a antiporter activity [GO:0015297]; is a type of secondary active monocarboxylate transmembrane transporter activity [GO:0015355] Also known as: glutamate-gamma-aminobutyric acid antiporter activity, glutamate/gamma-aminobutyric acid antiporter activity, glutamate: GABA antiporter activity Definition: Catalysis of the reaction: glutamate(out) + gamma-aminobutyric acid(in) = glutamate(in) + gamma-aminobutyric acid(out).